cuprous ion binding [GO:1903136] (molecular function) Relationships: is a type of copper ion binding [GO:0005507] Definition: Binding to a cuprous ion, copper(1+). References: PMID:24567322 Sources: GOC:PARL, GOC:TermGenie, GOC:bf, GO_REF:0000067 Also known as: Cu(+) binding, Cu(I) binding, copper(1+) binding